{
  "term_id": "GO:0005768",
  "gene_symbol": "SNX32",
  "gene": "UniProtKB:Q86XE0",
  "term_label": "endosome",
  "gene_name": "Sorting nexin-32"
}